{
  "gene_symbol": "ATP1B1",
  "term_id": "GO:0001671",
  "gene": "UniProtKB:P05026",
  "term_label": "ATPase activator activity",
  "gene_name": "Sodium_potassium-transporting ATPase subunit beta-1"
}